{
  "gene": "UniProtKB:Q9H598",
  "gene_name": "Vesicular inhibitory amino acid transporter",
  "term_id": "GO:0015812",
  "gene_symbol": "SLC32A1",
  "term_label": "gamma-aminobutyric acid transport"
}